{
  "gene_name": "Interleukin-13 receptor subunit alpha-2",
  "gene_symbol": "IL13RA2",
  "gene": "UniProtKB:Q14627",
  "term_id": "GO:0009897",
  "term_label": "external side of plasma membrane"
}